intrinsic apoptotic signaling pathway in response to oxidative stress [GO:0008631] (biological process) Relationships: is a type of intrinsic apoptotic signaling pathway [GO:0097193] Definition: The series of molecular signals in which an intracellular signal is conveyed to trigger the apoptotic death of a cell. The pathway is induced in response to oxidative stress, a state often resulting from exposure to high levels of reactive oxygen species, and ends when the execution phase of apoptosis is triggered. Regulation: regulated by GO:1902175; negatively regulated by negative regulation of oxidative stress-induced intrinsic apoptotic signaling pathway [GO:1902176]; RO_0002213 by positive regulation of oxidative stress-induced intrinsic apoptotic signaling pathway [GO:1902177] Sources: GOC:ai, GOC:mtg_apoptosis Also known as: oxidative stress-induced intrinsic apoptotic signaling pathway, induction of apoptosis by oxidative stress Subtypes: neuron intrinsic apoptotic signaling pathway in response to oxidative stress [GO:0036480], intrinsic apoptotic signaling pathway in response to hydrogen peroxide [GO:0036481]